negative regulation of L-glutamine biosynthetic process [GO:0062133] (biological process) References: PMID:19755423 Sources: GOC:ha Definition: Any process that stops, prevents or reduces the frequency, rate or extent of L-glutamine biosynthesis. Relationships: is a type of GO:0062014; is a type of regulation of L-glutamine biosynthetic process [GO:0062132]; is a type of GO:2000283; negatively regulates L-glutamine biosynthetic process [GO:1901704]